{
  "term_label": "regulation of cell population proliferation",
  "gene": "UniProtKB:P10600",
  "term_id": "GO:0042127",
  "gene_name": "Transforming growth factor beta-3 proprotein",
  "gene_symbol": "TGFB3"
}